{
  "gene": "UniProtKB:Q8NA19",
  "gene_symbol": "L3MBTL4",
  "term_id": "GO:0003682",
  "gene_name": "Lethal(3)malignant brain tumor-like protein 4",
  "term_label": "chromatin binding"
}